{
  "term_label": "L-ornithine transmembrane transporter activity",
  "term_id": "GO:0000064",
  "gene_symbol": "SLC7A2",
  "gene": "UniProtKB:P52569",
  "gene_name": "Cationic amino acid transporter 2"
}